{
  "term_id": "GO:0061575",
  "gene_symbol": "CCNT2",
  "gene": "UniProtKB:O60583",
  "term_label": "cyclin-dependent protein serine/threonine kinase activator activity",
  "gene_name": "Cyclin-T2"
}